{
  "gene_name": "Zona pellucida sperm-binding protein 3",
  "gene_symbol": "ZP3",
  "term_label": "egg coat formation",
  "gene": "UniProtKB:P21754",
  "term_id": "GO:0035803"
}